1-acylglycerophosphoserine O-acyltransferase activity [GO:0106263] (molecular function) References: PMID:18287005 Sources: RHEA:33191 Definition: Catalysis of the reaction:a 1-acyl-sn-glycero-3-phospho-L-serine + an acyl-CoA = a 1,2-diacyl-sn-glycero-3-phospho-L-serine + CoA. Relationships: is a type of GO:0008374